positive regulation of amacrine cell differentiation [GO:1902871] (biological process) Also known as: positive regulation of amacrine neuron differentiation, up regulation of amacrine cell differentiation, up regulation of amacrine neuron differentiation, up-regulation of amacrine cell differentiation, up-regulation of amacrine neuron differentiation, upregulation of amacrine cell differentiation, upregulation of amacrine neuron differentiation, activation of amacrine cell differentiation, activation of amacrine neuron differentiation References: PMID:16872597 Sources: GOC:TermGenie, GOC:mr, GO_REF:0000058 Definition: Any process that activates or increases the frequency, rate or extent of amacrine cell differentiation. Relationships: is a type of positive regulation of neuron differentiation [GO:0045666]; is a type of GO:1902869; positively regulates amacrine cell differentiation [GO:0035881]